{
  "term_label": "microtubule",
  "gene": "UniProtKB:P0DPH7",
  "gene_name": "Tubulin alpha-3C chain",
  "term_id": "GO:0005874",
  "gene_symbol": "TUBA3C"
}